(-)-exo-alpha-bergamotene biosynthetic process [GO:1901940] (biological process) Definition: The chemical reactions and pathways resulting in the formation of (-)-exo-alpha-bergamotene. References: PMID:22867794 Sources: GOC:TermGenie Also known as: (-)-exo-alpha-bergamotene anabolism, (-)-exo-alpha-bergamotene biosynthesis, (-)-exo-alpha-bergamotene formation, (-)-exo-alpha-bergamotene synthesis Relationships: is a type of sesquiterpene biosynthetic process [GO:0051762]; is a type of GO:1900674